D-lysopine dehydrogenase activity [GO:0047827] (molecular function) Relationships: is a type of oxidoreductase activity, acting on the CH-NH group of donors, NAD or NADP as acceptor [GO:0016646] Also known as: 2-N-(D-1-carboxyethyl)-L-lysine:NADP+ oxidoreductase (L-lysine-forming), D(+)-lysopine dehydrogenase activity, D-lysopine synthase activity, N2-(D-1-carboxyethyl)-L-lysine:NADP+ oxidoreductase (L-lysine-forming), lysopine dehydrogenase activity Sources: EC:1.5.1.16, RHEA:17625 Definition: Catalysis of the reaction: D-lysopine + H2O + NADP+ = L-lysine + H+ + NADPH + pyruvate.